{
  "gene": "UniProtKB:A6NC62",
  "term_label": "Unknown biological process",
  "gene_name": "Putative RBAK downstream neighbor protein",
  "gene_symbol": "RBAKDN",
  "term_id": "UNKNOWN:0002"
}